RNA methyltransferase activity [GO:0008173] (molecular function) Definition: Catalysis of the transfer of a methyl group from a donor to a nucleoside residue in an RNA molecule. Relationships: is a type of methyltransferase activity [GO:0008168]; is a type of GO:0140098 Sources: GOC:mah Subtypes: methyltransferase cap1 activity [GO:0004483], mRNA methyltransferase activity [GO:0008174], GO:0008175, GO:0008649, RNA 2'-O-methyltransferase activity [GO:0062105], RNA cap trimethylguanosine synthase activity [GO:0071164], snRNA methyltransferase activity [GO:0106346], GO:0120550, GO:1990276